{
  "gene_name": "Axin-2",
  "term_id": "GO:0005634",
  "gene": "UniProtKB:Q9Y2T1",
  "gene_symbol": "AXIN2",
  "term_label": "nucleus"
}